{
  "term_label": "nucleus",
  "gene_symbol": "UBE2Q1",
  "term_id": "GO:0005634",
  "gene": "UniProtKB:Q7Z7E8",
  "gene_name": "Ubiquitin-conjugating enzyme E2 Q1"
}